{
  "gene": "UniProtKB:Q8IYM9",
  "term_id": "GO:0032880",
  "gene_symbol": "TRIM22",
  "term_label": "regulation of protein localization",
  "gene_name": "E3 ubiquitin-protein ligase TRIM22"
}